{
  "term_id": "UNKNOWN:0002",
  "gene_symbol": "MZT2A",
  "gene_name": "Mitotic-spindle organizing protein 2A",
  "term_label": "Unknown biological process",
  "gene": "UniProtKB:Q6P582"
}